{
  "gene_name": "Ribonuclease P protein subunit p40",
  "term_label": "tRNA 5'-leader removal",
  "term_id": "GO:0001682",
  "gene_symbol": "RPP40",
  "gene": "UniProtKB:O75818"
}